{
  "term_label": "Notch binding",
  "gene_name": "Protein jagged-1",
  "gene": "UniProtKB:P78504",
  "term_id": "GO:0005112",
  "gene_symbol": "JAG1"
}